double membrane vesicle viral factory inner membrane [GO:0062245] (CC) Relationships: is a type of GO:0062242 Also known as: inner membrane of double membrane vesicle viral factory References: PMID:22440839 Definition: The inner of the two endoplasmic reticulum-derived lipid bilayer membranes that bound a double membrane vesicle viral factory.